{
  "term_label": "histone deacetylase complex",
  "gene": "UniProtKB:Q15652",
  "gene_symbol": "JMJD1C",
  "term_id": "GO:0000118",
  "gene_name": "Probable JmjC domain-containing histone demethylation protein 2C"
}